{
  "gene_name": "UDP-glucuronosyltransferase 2B28",
  "gene": "UniProtKB:Q9BY64",
  "gene_symbol": "UGT2B28",
  "term_label": "Unknown cellular component",
  "term_id": "UNKNOWN:0003"
}